{
  "term_id": "GO:0098839",
  "gene_symbol": "GRIN2D",
  "term_label": "postsynaptic density membrane",
  "gene": "UniProtKB:O15399",
  "gene_name": "Glutamate receptor ionotropic, NMDA 2D"
}